plant-type cell wall loosening [GO:0009828] (biological process) Also known as: cellulose and pectin-containing cell wall loosening Sources: GOC:lr, GOC:mtg_sensu Definition: The series of events causing chemical and structural alterations of an existing cellulose and pectin-containing cell wall that results in greater extensibility of the wall. An example of this is found in Arabidopsis thaliana. Relationships: is a type of plant-type cell wall modification [GO:0009827] Subtypes: plant-type cell wall loosening involved in abscission [GO:1902088]